glycosylated region protein binding [GO:0140081] (molecular function) Sources: GOC:pg Relationships: is a type of GO:0005515; is a type of carbohydrate derivative binding [GO:0097367] Definition: Binding to a glycosylated region of a protein.